{
  "term_id": "GO:0019432",
  "term_label": "triglyceride biosynthetic process",
  "gene_symbol": "LPIN2",
  "gene": "UniProtKB:Q92539",
  "gene_name": "Phosphatidate phosphatase LPIN2"
}